{
  "term_label": "beta-1,3-galactosyl-O-glycosyl-glycoprotein beta-1,3-N-acetylglucosaminyltransferase activity",
  "gene_name": "Protein O-linked-mannose beta-1,2-N-acetylglucosaminyltransferase 1",
  "gene": "UniProtKB:Q8WZA1",
  "term_id": "GO:0047223",
  "gene_symbol": "POMGNT1"
}